translation factor activity [GO:0180051] (molecular function) Sources: GOC:pg Relationships: is_a molecular_function [GO:0003674] Definition: A molecular function required for translation of a mRNA into a protein functioning as part of initiation, elongation or termination of translation. Subtypes: translation initiation factor activity [GO:0003743], GO:0003746, translation termination factor activity [GO:0008079], GO:0008135, translation factor activity, non-nucleic acid binding [GO:0045183]